{
  "gene": "UniProtKB:Q96PD2",
  "gene_symbol": "DCBLD2",
  "term_label": "plasma membrane",
  "gene_name": "Discoidin, CUB and LCCL domain-containing protein 2",
  "term_id": "GO:0005886"
}